{
  "gene": "UniProtKB:Q9NWL6",
  "term_id": "UNKNOWN:0001",
  "gene_name": "Asparagine synthetase domain-containing protein 1",
  "term_label": "Unknown molecular function",
  "gene_symbol": "ASNSD1"
}